{
  "gene": "UniProtKB:J3KSC0",
  "term_id": "UNKNOWN:0003",
  "term_label": "Unknown cellular component",
  "gene_symbol": "LINC01387",
  "gene_name": "Putative uncharacterized protein encoded by LINC01387"
}